N-acylneuraminate-9-phosphatase activity [GO:0050124] (molecular function) Definition: Catalysis of the reaction: N-acylneuraminate 9-phosphate + H2O = N-acylneuraminate + phosphate. Relationships: is_a phosphatase activity [GO:0016791] Sources: EC:3.1.3.29, MetaCyc:N-ACYLNEURAMINATE-9-PHOSPHATASE-RXN Also known as: N-acylneuraminate-9-phosphate phosphohydrolase activity, N-acylneuraminic (sialic) acid 9-phosphatase activity, N-acylneuraminic acid 9-phosphate phosphatase activity, acylneuraminate 9-phosphatase activity